regulation of ubiquitin-protein transferase activity [GO:0051438] (biological process) Relationships: is a type of GO:0051338; regulates ubiquitin-protein transferase activity [GO:0004842] Sources: GOC:ai, GOC:tb Subtypes: positive regulation of ubiquitin-protein transferase activity [GO:0051443], negative regulation of ubiquitin-protein transferase activity [GO:0051444], GO:1904666 Also known as: regulation of ubiquitin transferase activity, APC regulator, SCF complex regulator, anaphase-promoting complex regulator, ubiquitin transferase regulator, ubiquitin-protein transferase regulator Definition: Any process that modulates the frequency, rate or extent of ubiquitin transferase activity.